negative regulation of mitochondrial outer membrane permeabilization involved in apoptotic signaling pathway [GO:1901029] (biological process) Sources: GOC:BHF, GOC:TermGenie, GOC:mtg_apoptosis Relationships: is a type of negative regulation of organelle organization [GO:0010639]; is a type of negative regulation of mitochondrial membrane permeability [GO:0035795]; is a type of regulation of mitochondrial outer membrane permeabilization involved in apoptotic signaling pathway [GO:1901028]; is a type of GO:2001234; negatively regulates GO:0097345 Definition: Any process that stops, prevents or reduces the frequency, rate or extent of mitochondrial outer membrane permeabilization involved in apoptotic signaling pathway. Also known as: negative regulation of mitochondrial outer membrane permeabilization, down regulation of MOMP, down regulation of mitochondrial outer membrane permeabilization, down-regulation of MOMP, down-regulation of mitochondrial outer membrane permeabilization, downregulation of MOMP, downregulation of mitochondrial outer membrane permeabilization, negative regulation of MOMP, inhibition of MOMP, inhibition of mitochondrial outer membrane permeabilization